{
  "term_id": "UNKNOWN:0002",
  "gene_name": "von Willebrand factor A domain-containing protein 3A",
  "term_label": "Unknown biological process",
  "gene": "UniProtKB:A6NCI4",
  "gene_symbol": "VWA3A"
}